(1,4)-alpha-D-glucan 1-alpha-D-glucosylmutase activity [GO:0047470] (molecular function) Definition: Catalysis of the reaction: 4-[(1->4)-alpha-D-glucosyl](n-1)-D-glucose = 1-alpha-D-[(1->4)-alpha-D-glucosyl](n-1)-alpha-D-glucopyranoside. Sources: EC:5.4.99.15, MetaCyc:5.4.99.15-RXN Also known as: (1->4)-alpha-D-glucan 1-alpha-D-glucosylmutase, malto-oligosyltrehalose synthase activity, maltodextrin alpha-D-glucosyltransferase activity Relationships: is a type of intramolecular transferase activity [GO:0016866]